histone H3Y41 kinase activity [GO:0035401] (molecular function) Definition: Catalysis of the reaction: histone H3-tyrosine (position 41) + ATP = histone H3-phosphotyrosine (position 41) + ADP. This reaction is the addition of a phosphate group to the tyrosine residue at position 41 of histone H3. Relationships: is a type of GO:0004713; is a type of GO:0140996 Note: Comment: Note that the residue position corresponds to the canonical human H3 histone (UniProtKB:P84243); this residue is conserved across all eukaryotes. Residue 1 is the first residue following removal of the initiating Methionine (Met). Note that each histone is encoded by multiple genes, and sequences may vary across different genes within an organism. Also known as: histone H3-Y41 kinase activity, histone kinase activity (H3-Y41 specific), histone tyrosine kinase activity (H3-Y41 specific), histone-tyrosine kinase activity (H3-Y41 specific) Sources: GOC:bf